{
  "term_label": "telomere capping",
  "term_id": "GO:0016233",
  "gene_symbol": "POT1",
  "gene": "UniProtKB:Q9NUX5",
  "gene_name": "Protection of telomeres protein 1"
}